{
  "term_label": "immunoglobulin mediated immune response",
  "term_id": "GO:0016064",
  "gene": "UniProtKB:A0A0J9YY99",
  "gene_symbol": "A0A0J9YY99",
  "gene_name": "Ig-like domain-containing protein (Fragment)"
}